{
  "gene_symbol": "CENPI",
  "gene_name": "Centromere protein I",
  "term_id": "GO:0000939",
  "term_label": "inner kinetochore",
  "gene": "UniProtKB:Q92674"
}